{
  "gene_name": "Olfactory receptor 4D1",
  "gene": "UniProtKB:Q15615",
  "term_label": "plasma membrane",
  "gene_symbol": "OR4D1",
  "term_id": "GO:0005886"
}